{
  "term_id": "GO:0006887",
  "term_label": "exocytosis",
  "gene_name": "Putative WAS protein family homolog 3",
  "gene_symbol": "WASH3P",
  "gene": "UniProtKB:C4AMC7"
}